5(S)-hydroxyeicosatetraenoic acid dehydrogenase activity [GO:0097265] (molecular function) Definition: Catalysis of the reaction: 5-HETE + NADP+ = 5-oxo-ETE + NADPH + H+. Also known as: 5(S)-HETE dehydrogenase activity, 5-HETE dehydrogenase activity, 5-hydroxy-eicosatetraenoic acid dehydrogenase activity References: PMID:1326548 Sources: GOC:mw Relationships: is a type of oxidoreductase activity, acting on the CH-OH group of donors, NAD or NADP as acceptor [GO:0016616]